{
  "term_id": "GO:0004822",
  "term_label": "isoleucine-tRNA ligase activity",
  "gene_symbol": "IARS2",
  "gene_name": "Isoleucine--tRNA ligase, mitochondrial",
  "gene": "UniProtKB:Q9NSE4"
}